{
  "gene_name": "ATP synthase membrane subunit K, mitochondrial",
  "term_label": "Unknown molecular function",
  "gene": "UniProtKB:Q96IX5",
  "term_id": "UNKNOWN:0001",
  "gene_symbol": "ATP5MK"
}